{
  "gene_symbol": "IGHJ1",
  "term_id": "UNKNOWN:0003",
  "term_label": "Unknown cellular component",
  "gene": "UniProtKB:A0A0C4DH62",
  "gene_name": "Immunoglobulin heavy joining 1"
}